{
  "term_id": "GO:0098978",
  "gene": "UniProtKB:O60245",
  "term_label": "glutamatergic synapse",
  "gene_symbol": "PCDH7",
  "gene_name": "Protocadherin-7"
}